{
  "gene": "UniProtKB:Q13418",
  "gene_symbol": "ILK",
  "term_id": "GO:0005925",
  "gene_name": "Integrin-linked protein kinase",
  "term_label": "focal adhesion"
}